{
  "gene_symbol": "EDC3",
  "gene": "UniProtKB:Q96F86",
  "term_label": "deadenylation-independent decapping of nuclear-transcribed mRNA",
  "gene_name": "Enhancer of mRNA-decapping protein 3",
  "term_id": "GO:0031087"
}